{
  "gene": "UniProtKB:Q86UX7",
  "gene_symbol": "FERMT3",
  "gene_name": "Fermitin family homolog 3",
  "term_id": "GO:0033632",
  "term_label": "regulation of cell-cell adhesion mediated by integrin"
}